pattern specification involved in metanephros development [GO:0072268] (biological process) Definition: Any developmental process that results in the creation of defined areas or spaces within the metanephros to which cells respond and eventually are instructed to differentiate. Sources: GOC:mtg_kidney_jan10 Also known as: metanephros pattern specification, metanephros pattern formation, pattern formation involved in metanephros development Relationships: is a type of pattern specification involved in kidney development [GO:0061004]; is part of metanephros development [GO:0001656] Subtypes: GO:0072188, GO:0072267, GO:0072272, GO:0072293